{
  "gene_symbol": "ATP1B1",
  "gene_name": "Sodium_potassium-transporting ATPase subunit beta-1",
  "gene": "UniProtKB:P05026",
  "term_id": "GO:1990573",
  "term_label": "potassium ion import across plasma membrane"
}